{
  "gene": "UniProtKB:A6NFU0",
  "term_label": "Unknown biological process",
  "gene_symbol": "FAM187A",
  "term_id": "UNKNOWN:0002",
  "gene_name": "Ig-like V-type domain-containing protein FAM187A"
}